{
  "term_label": "endoplasmic reticulum membrane",
  "gene_name": "Protein ERGIC-53-like",
  "gene_symbol": "LMAN1L",
  "term_id": "GO:0005789",
  "gene": "UniProtKB:Q9HAT1"
}